{
  "term_id": "UNKNOWN:0001",
  "gene_name": "Hyaluronan and proteoglycan link protein 4",
  "term_label": "Unknown molecular function",
  "gene_symbol": "HAPLN4",
  "gene": "UniProtKB:Q86UW8"
}